determination of bilateral symmetry [GO:0009855] (biological process) Relationships: is a type of specification of symmetry [GO:0009799] Definition: The establishment of an organism's body plan or part of an organism with respect to a single longitudinal plane. The pattern can either be symmetric, such that the halves are mirror images, or asymmetric where the pattern deviates from this symmetry. Sources: GOC:go_curators Subtypes: determination of left/right symmetry [GO:0007368], determination of dorsal/ventral asymmetry [GO:0048262] Also known as: determination of bilateral asymmetry